{
  "gene_symbol": "ABT1",
  "gene": "UniProtKB:Q9ULW3",
  "gene_name": "Activator of basal transcription 1",
  "term_label": "RNA binding",
  "term_id": "GO:0003723"
}